cytosolic creatine kinase complex [GO:0002186] (cellular component) References: PMID:173175 Relationships: is a type of GO:0002185; is part of GO:0005829 Definition: A dimeric protein complex having creatine kinase activity.